{
  "term_label": "3'-UTR-mediated mRNA destabilization",
  "gene_symbol": "ZC3H12C",
  "gene_name": "Probable ribonuclease ZC3H12C",
  "term_id": "GO:0061158",
  "gene": "UniProtKB:Q9C0D7"
}